{
  "term_id": "GO:0000978",
  "gene_name": "Zinc finger protein 467",
  "term_label": "RNA polymerase II cis-regulatory region sequence-specific DNA binding",
  "gene_symbol": "ZNF467",
  "gene": "UniProtKB:Q7Z7K2"
}